{
  "term_id": "GO:0005794",
  "gene_symbol": "TMBIM1",
  "gene": "UniProtKB:Q969X1",
  "term_label": "Golgi apparatus",
  "gene_name": "Protein lifeguard 3"
}